{
  "gene_name": "Band 4.1-like protein 2",
  "gene": "UniProtKB:O43491",
  "term_id": "GO:0005856",
  "term_label": "cytoskeleton",
  "gene_symbol": "EPB41L2"
}